{
  "gene": "UniProtKB:O60941",
  "term_id": "GO:0099536",
  "term_label": "synaptic signaling",
  "gene_symbol": "DTNB",
  "gene_name": "Dystrobrevin beta"
}